{
  "term_label": "Unknown biological process",
  "gene": "UniProtKB:Q96NS5",
  "gene_symbol": "ASB16",
  "term_id": "UNKNOWN:0002",
  "gene_name": "Ankyrin repeat and SOCS box protein 16"
}